{
  "gene_symbol": "SELPLG",
  "gene_name": "P-selectin glycoprotein ligand 1",
  "term_id": "GO:0005886",
  "term_label": "plasma membrane",
  "gene": "UniProtKB:Q14242"
}